(R)-carnitine:4-(trimethylammonio)butanoate antiporter activity [GO:0044667] (molecular function) Definition: Enables the transfer of a solute or solutes from one side of a membrane to the other according to the reaction: (R)-carnitine(out) + 4-(trimethylammonio)butanoate(in) = (R)-carnitine(in) + 4-(trimethylammonio)butanoate(out). Sources: GOC:crds Also known as: (R)-carnitine:gamma-butyrobetaine antiporter activity, L-carnitine:4-(trimethylammonio)butanoate antiporter activity, L-carnitine:gamma-butyrobetaine antiporter activity Relationships: is_a antiporter activity [GO:0015297]; is a type of GO:1901235; is a type of 4-(trimethylammonio)butanoate transmembrane transporter activity [GO:1901236]